{
  "gene": "UniProtKB:P43631",
  "term_id": "GO:0005886",
  "gene_name": "Killer cell immunoglobulin-like receptor 2DS2",
  "term_label": "plasma membrane",
  "gene_symbol": "KIR2DS2"
}